{
  "gene_name": "BET1-like protein",
  "term_id": "GO:2000156",
  "term_label": "regulation of retrograde vesicle-mediated transport, Golgi to ER",
  "gene": "UniProtKB:Q9NYM9",
  "gene_symbol": "BET1L"
}